{
  "gene": "UniProtKB:A0A1B0GVM5",
  "gene_symbol": "ETDC",
  "term_label": "Unknown molecular function",
  "term_id": "UNKNOWN:0001",
  "gene_name": "Embryonic testis differentiation protein homolog C"
}